telencephalon oligodendrocyte cell migration [GO:0022032] (biological process) Definition: The multiplication or reproduction of telencephalon oligodendrocyte cells, resulting in the expansion of a cell population. Relationships: is a type of telencephalon glial cell migration [GO:0022030] Sources: GOC:cls, GOC:dgh, GOC:dph, GOC:jid, GO_REF:0000021